{
  "term_label": "succinyl-CoA metabolic process",
  "gene": "UniProtKB:Q96I99",
  "gene_symbol": "SUCLG2",
  "gene_name": "Succinate--CoA ligase [GDP-forming] subunit beta, mitochondrial",
  "term_id": "GO:0006104"
}